{
  "gene_name": "Zinc finger protein 623",
  "gene": "UniProtKB:O75123",
  "gene_symbol": "ZNF623",
  "term_label": "nucleus",
  "term_id": "GO:0005634"
}